{
  "term_id": "GO:0032797",
  "term_label": "SMN complex",
  "gene": "UniProtKB:Q8TEQ6",
  "gene_symbol": "GEMIN5",
  "gene_name": "Gem-associated protein 5"
}